2-hydroxy-6-oxonona-2,4,7-trienedioate hydrolase activity [GO:0052823] (molecular function) Also known as: (2E,4Z,7E)-2-hydroxy-6-oxonona-2,4,7-trienedioate fumarylhydrolase activity, 2-hydroxy-6-ketonona-2,4,7-trienedoic acid hydrolase activity Relationships: is a type of hydrolase activity, acting on acid carbon-carbon bonds, in ketonic substances [GO:0016823] Sources: RHEA:34191 Definition: Catalysis of the reaction: (2Z,4E,7E)-2-hydroxy-6-oxonona-2,4,7-trienedioate + H2O = (2Z)-2-hydroxypenta-2,4-dienoate + fumarate + H+.